{
  "gene_name": "Zinc finger protein 330",
  "term_label": "Unknown biological process",
  "gene": "UniProtKB:Q9Y3S2",
  "term_id": "UNKNOWN:0002",
  "gene_symbol": "ZNF330"
}